regulation of actin cytoskeleton organization by cell-cell adhesion [GO:0090138] (biological process) Relationships: is a type of regulation of actin cytoskeleton organization [GO:0032956]; is a type of cell-cell adhesion [GO:0098609] Also known as: regulation of actin cytoskeleton organisation by cell-cell adhesion Sources: GOC:ascb_2009, GOC:dph, GOC:tb Definition: Any cell-cell adhesion process that modulates the formation, arrangement of constituent parts, or disassembly of cytoskeletal structures comprising actin filaments and their associated proteins.